{
  "term_label": "G protein-coupled receptor signaling pathway",
  "term_id": "GO:0007186",
  "gene_name": "Olfactory receptor 5M9",
  "gene_symbol": "OR5M9",
  "gene": "UniProtKB:Q8NGP3"
}